{
  "term_label": "endoplasmic reticulum membrane",
  "gene_symbol": "ESYT2",
  "gene": "UniProtKB:A0FGR8",
  "gene_name": "Extended synaptotagmin-2",
  "term_id": "GO:0005789"
}